{
  "gene_name": "Eukaryotic translation initiation factor 4 gamma 1",
  "gene": "UniProtKB:Q04637",
  "term_label": "translation initiation factor activity",
  "term_id": "GO:0003743",
  "gene_symbol": "EIF4G1"
}